organ boundary specification between lateral organs and the meristem [GO:0010199] (BP) References: PMID:12068116 Definition: The process in which boundaries between lateral organs and the meristem is established and maintained. Relationships: is a type of GO:0090691